ciliary neurotrophic factor receptor activity [GO:0004897] (molecular function) Also known as: CNTF receptor activity, gp130 Subtypes: leukemia inhibitory factor receptor activity [GO:0004923] Definition: Combining with ciliary neurotrophic factor (CNTF) and transmitting the signal from one side of the membrane to the other to initiate a change in cell activity. Relationships: is a type of cytokine receptor activity [GO:0004896]; is part of ciliary neurotrophic factor-mediated signaling pathway [GO:0070120]; has part ciliary neurotrophic factor binding [GO:0070119] Sources: GOC:mah, GOC:signaling